symplast [GO:0055044] (cellular component) Definition: The interconnected cell membranes and intracellular regions of a plant. The interconnections occur via the plasmodesmata. Sources: GOC:mtg_sensu Relationships: is a type of GO:0110165